D-amino-acid dehydrogenase complex [GO:0009324] (cellular component) Note: See also the molecular function term 'D-amino-acid oxidase activity ; GO:0003884'. Definition: A protein complex that possesses D-amino-acid dehydrogenase activity. Relationships: is a type of GO:0098797; is a type of oxidoreductase complex [GO:1990204] Sources: GOC:mah